supercoiled DNA binding [GO:0097100] (molecular function) Definition: Binding to supercoiled DNA. For example, during replication and transcription, template DNA is negatively supercoiled in the receding downstream DNA and positively supercoiled in the approaching downstream DNA. References: PMID:20723754, PMID:21345933 Sources: GOC:pr, GOC:rph, Wikipedia:DNA_supercoil Relationships: is a type of double-stranded DNA binding [GO:0003690]